peroxisomal membrane [GO:0005778] (cellular component) Relationships: is a type of microbody membrane [GO:0031903]; is part of GO:0005777 Subtypes: GO:0046860, glyoxysomal membrane [GO:0046861] Sources: GOC:mah Also known as: peroxisome membrane Definition: The lipid bilayer surrounding a peroxisome.